{
  "gene_symbol": "TRAJ19",
  "gene": "UniProtKB:A0A075B6Y4",
  "gene_name": "T cell receptor alpha joining 19 (non-functional) (Fragment)",
  "term_id": "UNKNOWN:0003",
  "term_label": "Unknown cellular component"
}